regulation of mitotic cytokinetic process [GO:1903436] (biological process) Definition: Any process that modulates the frequency, rate or extent of mitotic cytokinetic process. Sources: GOC:TermGenie, GOC:vw, GO_REF:0000058 Relationships: is a type of regulation of cytokinetic process [GO:0032954]; is a type of regulation of mitotic cytokinesis [GO:1902412]; regulates mitotic cytokinetic process [GO:1902410] Subtypes: GO:0140279, regulation of mitotic cytokinesis, division site positioning [GO:1902472], regulation of secondary cell septum biogenesis [GO:1903395], negative regulation of mitotic cytokinetic process [GO:1903437], positive regulation of mitotic cytokinetic process [GO:1903438], regulation of mitotic actomyosin contractile ring contraction [GO:1903471], regulation of mitotic actomyosin contractile ring assembly [GO:1903499]